{
  "gene_symbol": "SPRR2A",
  "term_label": "defense response to Gram-positive bacterium",
  "gene": "UniProtKB:P35326",
  "gene_name": "Small proline-rich protein 2A",
  "term_id": "GO:0050830"
}